{
  "term_label": "steroid hydroxylase activity",
  "gene_symbol": "CYP1A2",
  "term_id": "GO:0008395",
  "gene_name": "Cytochrome P450 1A2",
  "gene": "UniProtKB:P05177"
}